{
  "term_label": "peroxisome fission",
  "gene_symbol": "PEX11A",
  "term_id": "GO:0016559",
  "gene_name": "Peroxisomal membrane protein 11A",
  "gene": "UniProtKB:O75192"
}